{
  "gene_symbol": "PPT2",
  "term_id": "GO:0005764",
  "gene": "UniProtKB:Q9UMR5",
  "gene_name": "Lysosomal thioesterase PPT2",
  "term_label": "lysosome"
}